nuatigenin 3-beta-glucosyltransferase activity [GO:0047248] (molecular function) Definition: Catalysis of the reaction: nuatigenin + UDP-D-glucose = H+ + nuatigenin 3-beta-D-glucopyranoside + UDP. Relationships: is a type of UDP-glucosyltransferase activity [GO:0035251] Also known as: UDP-glucose:(20S,22S,25S)-22,25-epoxyfurost-5-ene-3beta,26-diol 3-O-beta-D-glucosyltransferase activity, UDPglucose:(20S,22S,25S)-22,25-epoxyfurost-5-ene-3beta,26-diol 3-O-beta-D-glucosyltransferase activity, nuatigenin 3beta-glucosyltransferase activity, uridine diphosphoglucose-nuatigenin glucosyltransferase activity Sources: EC:2.4.1.192, RHEA:19329